{
  "gene_symbol": "ECSIT",
  "term_id": "GO:0045087",
  "term_label": "innate immune response",
  "gene_name": "Evolutionarily conserved signaling intermediate in Toll pathway, mitochondrial",
  "gene": "UniProtKB:Q9BQ95"
}